{
  "term_id": "GO:0007155",
  "term_label": "cell adhesion",
  "gene_name": "Intercellular adhesion molecule 2",
  "gene": "UniProtKB:P13598",
  "gene_symbol": "ICAM2"
}